{
  "term_id": "UNKNOWN:0001",
  "gene_name": "Ankyrin repeat and SOCS box protein 13",
  "term_label": "Unknown molecular function",
  "gene_symbol": "ASB13",
  "gene": "UniProtKB:Q8WXK3"
}